{
  "gene": "UniProtKB:A0A1B0GVH4",
  "gene_symbol": "PRSS51",
  "term_id": "GO:0016485",
  "gene_name": "Serine protease-like protein 51",
  "term_label": "protein processing"
}